{
  "gene_name": "EH domain-containing protein 1",
  "term_label": "recycling endosome membrane",
  "gene": "UniProtKB:Q9H4M9",
  "term_id": "GO:0055038",
  "gene_symbol": "EHD1"
}